{
  "term_label": "U4/U6 x U5 tri-snRNP complex",
  "gene_name": "Pre-mRNA-splicing factor 18",
  "term_id": "GO:0046540",
  "gene_symbol": "PRPF18",
  "gene": "UniProtKB:Q99633"
}